{
  "gene": "UniProtKB:Q8TDN2",
  "term_id": "GO:0001508",
  "gene_symbol": "KCNV2",
  "term_label": "action potential",
  "gene_name": "Potassium voltage-gated channel subfamily V member 2"
}